{
  "gene": "UniProtKB:P0DP03",
  "gene_name": "Immunoglobulin heavy variable 3-30-5",
  "term_label": "Unknown cellular component",
  "gene_symbol": "IGHV3-30-5",
  "term_id": "UNKNOWN:0003"
}